{
  "gene_symbol": "CCPG1",
  "term_id": "GO:0016020",
  "gene_name": "Cell cycle progression protein 1",
  "term_label": "membrane",
  "gene": "UniProtKB:Q9ULG6"
}